{
  "term_id": "GO:0019901",
  "term_label": "protein kinase binding",
  "gene_name": "E3 ubiquitin-protein ligase TRIM22",
  "gene": "UniProtKB:Q8IYM9",
  "gene_symbol": "TRIM22"
}